{
  "term_label": "neuropeptide signaling pathway",
  "gene_name": "Neuropeptide FF receptor 1",
  "gene": "UniProtKB:Q9GZQ6",
  "gene_symbol": "NPFFR1",
  "term_id": "GO:0007218"
}